{
  "gene_symbol": "IL1RAP",
  "term_label": "cell surface",
  "term_id": "GO:0009986",
  "gene": "UniProtKB:Q9NPH3",
  "gene_name": "Interleukin-1 receptor accessory protein"
}